{
  "gene_symbol": "OR1L6",
  "term_label": "olfactory receptor activity",
  "term_id": "GO:0004984",
  "gene_name": "Olfactory receptor 1L6",
  "gene": "UniProtKB:Q8NGR2"
}